estrogen 16-alpha-hydroxylase activity [GO:0101020] (molecular function) Definition: Catalysis of the reaction: estrogen + reduced [NADPH--hemoprotein reductase] + O2 = 16-alpha-hydroxyestrogen + oxidized [NADPH--hemoprotein reductase] + H2O. Sources: GOC:BHF Also known as: oestrogen 16-alpha-hydroxylase activity Relationships: is a type of GO:0008395; is a type of oxidoreductase activity, acting on paired donors, with incorporation or reduction of molecular oxygen, reduced flavin or flavoprotein as one donor, and incorporation of one atom of oxygen [GO:0016712]